RNA endonuclease activity producing 5'-phosphomonoesters, hydrolytic mechanism [GO:0016891] (molecular function) Definition: Catalysis of the hydrolysis of ester linkages within ribonucleic acids by creating internal breaks to yield 5'-phosphomonoesters. Relationships: is a type of RNA endonuclease activity [GO:0004521]; is a type of hydrolase activity, acting on ester bonds [GO:0016788] Subtypes: GO:0004523, GO:0004525, ribonuclease P activity [GO:0004526], RNA lariat debranching enzyme activity [GO:0008419], ribonuclease E activity [GO:0008995], ribonuclease IV activity [GO:0033893], ribonuclease P4 activity [GO:0033894], ribonuclease [poly-(U)-specific] activity [GO:0033895], GO:0033896, 3'-tRNA processing endoribonuclease activity [GO:0042781], GO:0043822, RNA-(apurinic or apyrimidinic site) endonuclease activity [GO:0052719], endoribonuclease activity, cleaving siRNA-paired mRNA [GO:0070551], endoribonuclease activity, cleaving miRNA-paired mRNA [GO:0090624], phosphodiesterase decapping endonuclease activity [GO:1990174] Also known as: endoribonuclease activity, producing 5'-phosphomonoesters Sources: GOC:ai